{
  "gene_symbol": "MDH2",
  "gene": "UniProtKB:P40926",
  "gene_name": "Malate dehydrogenase, mitochondrial",
  "term_label": "mitochondrion",
  "term_id": "GO:0005739"
}